{
  "gene_symbol": "GABARAP",
  "gene": "UniProtKB:O95166",
  "term_id": "GO:0008429",
  "term_label": "phosphatidylethanolamine binding",
  "gene_name": "Gamma-aminobutyric acid receptor-associated protein"
}